{
  "gene_symbol": "RPGRIP1",
  "gene_name": "X-linked retinitis pigmentosa GTPase regulator-interacting protein 1",
  "term_id": "GO:0046548",
  "gene": "UniProtKB:Q96KN7",
  "term_label": "retinal rod cell development"
}